{
  "gene_symbol": "CLEC19A",
  "gene_name": "C-type lectin domain family 19 member A",
  "term_id": "UNKNOWN:0001",
  "term_label": "Unknown molecular function",
  "gene": "UniProtKB:Q6UXS0"
}